{
  "gene_name": "Synaptotagmin-6",
  "gene_symbol": "SYT6",
  "term_id": "GO:0007268",
  "term_label": "chemical synaptic transmission",
  "gene": "UniProtKB:Q5T7P8"
}